{
  "gene_name": "WD repeat and FYVE domain-containing protein 2",
  "gene": "UniProtKB:Q96P53",
  "term_id": "GO:0045600",
  "gene_symbol": "WDFY2",
  "term_label": "positive regulation of fat cell differentiation"
}